{
  "term_id": "GO:0009888",
  "gene_name": "Steroidogenic factor 1",
  "term_label": "tissue development",
  "gene": "UniProtKB:Q13285",
  "gene_symbol": "NR5A1"
}